regulation of adaptive immune effector response [GO:1905677] (biological process) Definition: Any process that modulates the frequency, rate or extent of adaptive immune effector response. Sources: GOC:TermGenie, GO_REF:0000058, ISBN:9781405196833 Relationships: is a type of regulation of adaptive immune response [GO:0002819]; regulates GO:0090718 Subtypes: GO:1905678, positive regulation of adaptive immune effector response [GO:1905679]